{
  "term_label": "extracellular space",
  "term_id": "GO:0005615",
  "gene_name": "Inhibin alpha chain",
  "gene": "UniProtKB:P05111",
  "gene_symbol": "INHA"
}